{
  "gene_symbol": "PGK1",
  "term_id": "GO:0005524",
  "gene": "UniProtKB:P00558",
  "term_label": "ATP binding",
  "gene_name": "Phosphoglycerate kinase 1"
}